{
  "gene_name": "EKC_KEOPS complex subunit TP53RK",
  "term_label": "EKC/KEOPS complex",
  "gene": "UniProtKB:Q96S44",
  "gene_symbol": "TP53RK",
  "term_id": "GO:0000408"
}